sensory processing [GO:0050893] (biological process) Relationships: is a type of cognition [GO:0050890]; is part of sensory perception [GO:0007600] Sources: GOC:dph, ISBN:0721662544 Definition: Any neural process required for an organism to sense and interpret the dimensions of a sensory experience: modality, location, intensity and affect. Subtypes: determination of sensory modality [GO:0050887], determination of stimulus location [GO:0050888], determination of stimulus intensity [GO:0050889], GO:0050894